cardiac chamber formation [GO:0003207] (biological process) Sources: GOC:mtg_heart Also known as: heart chamber formation Regulation: regulated by GO:1901210; negatively regulated by negative regulation of cardiac chamber formation [GO:1901211]; positively regulated by positive regulation of cardiac chamber formation [GO:1901212] Definition: The developmental process pertaining to the initial formation of a cardiac chamber from unspecified parts. A cardiac chamber is an enclosed cavity within the heart. Subtypes: cardiac atrium formation [GO:0003210], GO:0003211, bulbus arteriosus formation [GO:0003234], sinus venosus formation [GO:0003237], conus arteriosus formation [GO:0003240] Relationships: is a type of anatomical structure formation involved in morphogenesis [GO:0048646]; is part of cardiac chamber morphogenesis [GO:0003206]